tRNA threonylcarbamoyladenosine metabolic process [GO:0070525] (BP) Relationships: is a type of tRNA metabolic process [GO:0006399] Subtypes: tRNA threonylcarbamoyladenosine modification [GO:0002949], GO:0070900 Also known as: t6A metabolic process, t6A metabolism, threonylcarbamoyladenosine metabolism Definition: The chemical reactions and pathways involving tRNA threonylcarbamoyladenosine, a modified nucleoside found in some tRNA molecules. References: PMID:19287007 Sources: GOC:imk, GOC:mah